glucosamine-containing compound biosynthetic process [GO:1901073] (biological process) Relationships: is_a GO:0046349 Sources: GOC:TermGenie Subtypes: chitin biosynthetic process [GO:0006031], glucosamine biosynthetic process [GO:0006042], N-acetylglucosamine biosynthetic process [GO:0006045] Also known as: glucosamine-containing compound anabolism, glucosamine-containing compound biosynthesis, glucosamine-containing compound formation, glucosamine-containing compound synthesis, glucosamines anabolism, glucosamines biosynthesis, glucosamines biosynthetic process, glucosamines formation, glucosamines synthesis Definition: The chemical reactions and pathways resulting in the formation of glucosamine-containing compounds (glucosamines).